{
  "term_label": "immune response",
  "term_id": "GO:0006955",
  "gene_name": "Transforming growth factor beta activator LRRC33",
  "gene": "UniProtKB:Q86YC3",
  "gene_symbol": "NRROS"
}